{
  "term_label": "ionotropic glutamate receptor binding",
  "term_id": "GO:0035255",
  "gene_name": "Protein shisa-6",
  "gene": "UniProtKB:Q6ZSJ9",
  "gene_symbol": "SHISA6"
}